regulation of thylakoid membrane disassembly [GO:0010548] (biological process) Definition: Any process that modulates the frequency, rate or extent of thylakoid membrane disassembly. Also known as: regulation of thylakoid membrane degradation Relationships: is a type of regulation of membrane disassembly [GO:0010549]; regulates thylakoid membrane disassembly [GO:0010547] References: PMID:17416733 Sources: GOC:dph, GOC:tb